{
  "gene": "UniProtKB:P62249",
  "term_label": "maturation of SSU-rRNA from tricistronic rRNA transcript (SSU-rRNA, 5.8S rRNA, LSU-rRNA)",
  "gene_name": "Small ribosomal subunit protein uS9",
  "gene_symbol": "RPS16",
  "term_id": "GO:0000462"
}